{
  "gene": "UniProtKB:Q5VST6",
  "term_id": "GO:0099175",
  "gene_name": "Alpha_beta hydrolase domain-containing protein 17B",
  "term_label": "regulation of postsynapse organization",
  "gene_symbol": "ABHD17B"
}